{
  "term_id": "GO:0005200",
  "gene": "UniProtKB:P0DPH8",
  "term_label": "structural constituent of cytoskeleton",
  "gene_symbol": "TUBA3D",
  "gene_name": "Tubulin alpha-3D chain"
}